{
  "term_label": "cellular response to zinc ion",
  "gene_name": "Metallothionein 1H-like protein 1",
  "gene_symbol": "MT1HL1",
  "gene": "UniProtKB:P0DM35",
  "term_id": "GO:0071294"
}